{
  "gene_name": "CUB domain-containing protein",
  "term_id": "UNKNOWN:0003",
  "gene": "UniProtKB:A0A494C103",
  "gene_symbol": "SPADH",
  "term_label": "Unknown cellular component"
}